{
  "gene_name": "Ubiquitin carboxyl-terminal hydrolase 14",
  "term_id": "GO:1904293",
  "gene": "UniProtKB:P54578",
  "gene_symbol": "USP14",
  "term_label": "negative regulation of ERAD pathway"
}